negative regulation of methyl-branched fatty acid biosynthetic process [GO:1902323] (biological process) References: PMID:15340492 Sources: GOC:TermGenie, GOC:kmv Relationships: is a type of GO:0045717; is a type of GO:1902322; negatively regulates methyl-branched fatty acid biosynthetic process [GO:1902321] Also known as: down regulation of methyl-branched fatty acid anabolism, down regulation of methyl-branched fatty acid biosynthesis, down regulation of methyl-branched fatty acid biosynthetic process, down regulation of methyl-branched fatty acid formation, down regulation of methyl-branched fatty acid synthesis, down-regulation of methyl-branched fatty acid anabolism, down-regulation of methyl-branched fatty acid biosynthesis, down-regulation of methyl-branched fatty acid biosynthetic process, down-regulation of methyl-branched fatty acid formation, down-regulation of methyl-branched fatty acid synthesis, downregulation of methyl-branched fatty acid anabolism, downregulation of methyl-branched fatty acid biosynthesis, downregulation of methyl-branched fatty acid biosynthetic process, downregulation of methyl-branched fatty acid formation, downregulation of methyl-branched fatty acid synthesis, negative regulation of methyl-branched fatty acid anabolism, negative regulation of methyl-branched fatty acid biosynthesis, negative regulation of methyl-branched fatty acid formation, negative regulation of methyl-branched fatty acid synthesis, inhibition of methyl-branched fatty acid anabolism, inhibition of methyl-branched fatty acid biosynthesis, inhibition of methyl-branched fatty acid biosynthetic process, inhibition of methyl-branched fatty acid formation, inhibition of methyl-branched fatty acid synthesis Definition: Any process that stops, prevents or reduces the frequency, rate or extent of methyl-branched fatty acid biosynthetic process.